nicotianamine aminotransferase activity [GO:0033855] (molecular function) Relationships: is_a transaminase activity [GO:0008483] Sources: EC:2.6.1.80, RHEA:22104 Definition: Catalysis of the reaction: 2-oxoglutarate + nicotianamine = 3''-deamino-3''-oxonicotianamine + L-glutamate. Also known as: NAAT, NAAT-I, NAAT-II, NAAT-III, nicotianamine transaminase activity, nicotianamine:2-oxoglutarate aminotransferase activity